{
  "term_id": "UNKNOWN:0001",
  "gene_name": "BLOC-2 complex member HPS5",
  "gene": "UniProtKB:Q9UPZ3",
  "term_label": "Unknown molecular function",
  "gene_symbol": "HPS5"
}